{
  "term_id": "UNKNOWN:0002",
  "gene_name": "Olfactory receptor 14C36",
  "gene": "UniProtKB:Q8NHC7",
  "term_label": "Unknown biological process",
  "gene_symbol": "OR14C36"
}